{
  "term_id": "GO:0006612",
  "gene_name": "Golgin subfamily A member 7",
  "term_label": "protein targeting to membrane",
  "gene_symbol": "GOLGA7",
  "gene": "UniProtKB:Q7Z5G4"
}